{
  "gene": "UniProtKB:Q9H3U7",
  "gene_symbol": "SMOC2",
  "gene_name": "SPARC-related modular calcium-binding protein 2",
  "term_label": "heparin binding",
  "term_id": "GO:0008201"
}